{
  "gene_name": "Melanoma-associated antigen D2",
  "gene": "UniProtKB:Q9UNF1",
  "gene_symbol": "MAGED2",
  "term_label": "nucleus",
  "term_id": "GO:0005634"
}